{
  "gene_name": "T-cell surface glycoprotein CD3 gamma chain",
  "gene": "UniProtKB:P09693",
  "term_label": "cell surface receptor signaling pathway",
  "term_id": "GO:0007166",
  "gene_symbol": "CD3G"
}